{
  "gene": "UniProtKB:Q13367",
  "term_id": "UNKNOWN:0003",
  "gene_name": "AP-3 complex subunit beta-2",
  "gene_symbol": "AP3B2",
  "term_label": "Unknown cellular component"
}